{
  "gene": "UniProtKB:Q8IYS0",
  "gene_symbol": "GRAMD1C",
  "term_label": "cholesterol transfer activity",
  "term_id": "GO:0120020",
  "gene_name": "Protein Aster-C"
}